{
  "gene": "UniProtKB:P01034",
  "gene_symbol": "CST3",
  "term_id": "GO:0004869",
  "gene_name": "Cystatin-C",
  "term_label": "cysteine-type endopeptidase inhibitor activity"
}